spindle disassembly [GO:0051230] (biological process) Also known as: spindle breakdown, spindle catabolism, spindle degradation Sources: GOC:ai Subtypes: mitotic spindle disassembly [GO:0051228], GO:0051229 Definition: The controlled breakdown of the spindle, the array of microtubules and associated molecules that serves to move duplicated chromosomes apart. Relationships: is a type of GO:0007051; is a type of organelle disassembly [GO:1903008]